{
  "gene_name": "Transmembrane protein 273",
  "gene": "UniProtKB:Q5T292",
  "term_label": "Unknown biological process",
  "term_id": "UNKNOWN:0002",
  "gene_symbol": "TMEM273"
}